{
  "term_id": "GO:0000786",
  "gene_symbol": "H2BC5",
  "gene_name": "Histone H2B type 1-D",
  "gene": "UniProtKB:P58876",
  "term_label": "nucleosome"
}